{
  "gene_symbol": "HEBP2",
  "gene_name": "Heme-binding protein 2",
  "gene": "UniProtKB:Q9Y5Z4",
  "term_label": "Unknown biological process",
  "term_id": "UNKNOWN:0002"
}